{
  "gene": "UniProtKB:Q9Y4E6",
  "gene_symbol": "WDR7",
  "term_label": "Unknown biological process",
  "gene_name": "WD repeat-containing protein 7",
  "term_id": "UNKNOWN:0002"
}